{
  "gene": "UniProtKB:Q5VUJ9",
  "gene_name": "Dynein regulatory complex protein 8",
  "gene_symbol": "EFCAB2",
  "term_label": "Unknown molecular function",
  "term_id": "UNKNOWN:0001"
}